{
  "gene_symbol": "UBXN2B",
  "gene": "UniProtKB:Q14CS0",
  "term_id": "GO:0005634",
  "term_label": "nucleus",
  "gene_name": "UBX domain-containing protein 2B"
}